{
  "gene_symbol": "SLC16A8",
  "term_label": "plasma membrane",
  "term_id": "GO:0005886",
  "gene_name": "Monocarboxylate transporter 3",
  "gene": "UniProtKB:O95907"
}